{
  "term_label": "immune response-activating signaling pathway",
  "term_id": "GO:0002757",
  "gene": "UniProtKB:A8K4G0",
  "gene_symbol": "CD300LB",
  "gene_name": "CMRF35-like molecule 7"
}